{
  "gene_symbol": "BEX5",
  "gene": "UniProtKB:Q5H9J7",
  "gene_name": "Protein BEX5",
  "term_id": "GO:0005737",
  "term_label": "cytoplasm"
}